regulation of mesonephric glomerulus development [GO:2000087] (biological process) Sources: GOC:mtg_kidney_jan10 Subtypes: GO:2000088, GO:2000089 Relationships: is a type of regulation of mesonephros development [GO:0061217]; is a type of regulation of glomerulus development [GO:0090192]; regulates mesonephric glomerulus development [GO:0061224] Definition: Any process that modulates the frequency, rate or extent of mesonephric glomerulus development.